{
  "gene": "UniProtKB:O95210",
  "term_id": "UNKNOWN:0001",
  "term_label": "Unknown molecular function",
  "gene_name": "Starch-binding domain-containing protein 1",
  "gene_symbol": "STBD1"
}